modulation of spore encystment on host [GO:0075215] (biological process) Subtypes: positive regulation of spore encystment on host [GO:0075216], negative regulation of spore encystment on host [GO:0075217], modulation of zoospore encystment on host [GO:0075219] Sources: GOC:pamgo_curators Definition: Any process that modulates the frequency, rate or extent of spore encystment on host. The host is defined as the larger of the organisms involved in a symbiotic interaction. Relationships: is a type of regulation of cell development [GO:0060284]; regulates spore encystment [GO:0075214]